regulation of cardiac muscle tissue regeneration [GO:1905178] (biological process) References: PMID:23222520 Sources: GOC:BHF, GOC:BHF_miRNA, GOC:TermGenie, GOC:rph, GO_REF:0000058 Subtypes: negative regulation of cardiac muscle tissue regeneration [GO:1905179], positive regulation of cardiac muscle tissue regeneration [GO:1905180] Relationships: is a type of regulation of developmental growth [GO:0048638]; regulates GO:0061026 Definition: Any process that modulates the frequency, rate or extent of cardiac muscle tissue regeneration.